{
  "term_label": "endocytic vesicle",
  "gene_symbol": "VPS9D1",
  "gene_name": "VPS9 domain-containing protein 1",
  "term_id": "GO:0030139",
  "gene": "UniProtKB:Q9Y2B5"
}